epsilon DNA polymerase complex [GO:0008622] (cellular component) Relationships: is a type of DNA polymerase complex [GO:0042575]; is a type of nuclear protein-containing complex [GO:0140513]; is part of GO:0000228 Also known as: DNA polymerase epsilon complex Definition: A heterotetrameric DNA polymerase complex that catalyzes processive DNA synthesis in the absence of PCNA, but is further stimulated in the presence of PCNA. The complex contains a large catalytic subunit and three small subunits, and is best characterized in Saccharomyces, in which the subunits are named Pol2p, Dpb2p, Dpb3p, and Dpb4p. Some evidence suggests that DNA polymerase epsilon is the leading strand polymerase; it is also involved in nucleotide-excision repair and mismatch repair. References: PMID:15814431, PMID:9745046